regulation of post-translational protein modification [GO:1901873] (biological process) Relationships: is a type of GO:0031399; regulates post-translational protein modification [GO:0043687] References: PMID:21209915 Sources: GOC:TermGenie, GOC:yaf Subtypes: GO:1901874, GO:1901875, regulation of protein modification by small protein conjugation or removal [GO:1903320] Also known as: regulation of PTM, regulation of post-translational amino acid modification, regulation of post-translational modification, regulation of posttranslational amino acid modification, regulation of posttranslational modification, regulation of posttranslational protein modification Definition: Any process that modulates the frequency, rate or extent of post-translational protein modification.